{
  "gene_symbol": "PHF10",
  "gene": "UniProtKB:Q8WUB8",
  "term_id": "GO:0003712",
  "term_label": "transcription coregulator activity",
  "gene_name": "PHD finger protein 10"
}